smooth muscle contraction [GO:0006939] (biological process) Sources: GOC:ef, GOC:jl, GOC:mtg_muscle, ISBN:0198506732 Relationships: is a type of GO:0006936 Definition: A process in which force is generated within smooth muscle tissue, resulting in a change in muscle geometry. Force generation involves a chemo-mechanical energy conversion step that is carried out by the actin/myosin complex activity, which generates force through ATP hydrolysis. Smooth muscle differs from striated muscle in the much higher actin/myosin ratio, the absence of conspicuous sarcomeres and the ability to contract to a much smaller fraction of its resting length. Also known as: visceral muscle contraction Subtypes: tonic smooth muscle contraction [GO:0014820], phasic smooth muscle contraction [GO:0014821], vascular associated smooth muscle contraction [GO:0014829], gastro-intestinal system smooth muscle contraction [GO:0014831], GO:0014848, hindgut contraction [GO:0043133], uterine smooth muscle contraction [GO:0070471], colon smooth muscle contraction [GO:1990765], small intestine smooth muscle contraction [GO:1990770] Regulation: regulated by regulation of smooth muscle contraction [GO:0006940]; negatively regulated by negative regulation of smooth muscle contraction [GO:0045986]; positively regulated by positive regulation of smooth muscle contraction [GO:0045987]